{
  "term_id": "GO:0090161",
  "term_label": "Golgi ribbon formation",
  "gene_name": "Optineurin",
  "gene_symbol": "OPTN",
  "gene": "UniProtKB:Q96CV9"
}